{
  "gene_symbol": "CLCN3",
  "gene_name": "H(+)_Cl(-) exchange transporter 3",
  "gene": "UniProtKB:P51790",
  "term_label": "plasma membrane",
  "term_id": "GO:0005886"
}